{
  "term_id": "GO:0051726",
  "gene_symbol": "GADD45B",
  "term_label": "regulation of cell cycle",
  "gene_name": "Growth arrest and DNA damage-inducible protein GADD45 beta",
  "gene": "UniProtKB:O75293"
}